{
  "term_label": "Unknown molecular function",
  "gene_symbol": "MAGEB2",
  "gene_name": "Melanoma-associated antigen B2",
  "term_id": "UNKNOWN:0001",
  "gene": "UniProtKB:O15479"
}